{
  "term_label": "Unknown biological process",
  "term_id": "UNKNOWN:0002",
  "gene": "UniProtKB:Q86WB7",
  "gene_name": "Protein unc-93 homolog A",
  "gene_symbol": "UNC93A"
}